{
  "term_label": "adherens junction",
  "gene": "UniProtKB:Q8IXH8",
  "term_id": "GO:0005912",
  "gene_name": "Cadherin-like protein 26",
  "gene_symbol": "CDH26"
}